corpora quadrigemina development [GO:0061378] (biological process) Definition: The progression of the corpora quadrigemina over time, from its formation to the mature structure. The corpora quadrigemina is a part of the midbrain that is made up of the superior and inferior colliculi. Sources: GOC:dph, GOC:yaf Relationships: is a type of GO:0048856; is part of GO:0030901